{
  "gene": "UniProtKB:P43007",
  "term_label": "L-aspartate transmembrane transporter activity",
  "gene_symbol": "SLC1A4",
  "term_id": "GO:0015183",
  "gene_name": "Neutral amino acid transporter A"
}